negative regulation of protein localization to microtubule [GO:1902817] (biological process) References: PMID:23087209 Sources: GOC:TermGenie, GOC:vw, GO_REF:0000058 Relationships: is_a regulation of protein localization to microtubule [GO:1902816]; is a type of negative regulation of protein localization [GO:1903828]; negatively regulates protein localization to microtubule [GO:0035372] Definition: Any process that stops, prevents or reduces the frequency, rate or extent of protein localization to microtubule. Also known as: down regulation of protein localisation to microtubule, down regulation of protein localization to microtubule, down-regulation of protein localisation to microtubule, down-regulation of protein localization to microtubule, downregulation of protein localisation to microtubule, downregulation of protein localization to microtubule, negative regulation of protein localisation to microtubule, inhibition of protein localisation to microtubule, inhibition of protein localization to microtubule